A1 adenosine receptor binding [GO:0031686] (molecular function) Definition: Binding to an A1 adenosine receptor. Sources: GOC:mah, GOC:nln Relationships: is a type of adenosine receptor binding [GO:0031685] Also known as: A1 adenosine receptor ligand